regulation of striated muscle cell apoptotic process [GO:0010662] (biological process) Subtypes: positive regulation of striated muscle cell apoptotic process [GO:0010663], negative regulation of striated muscle cell apoptotic process [GO:0010664], regulation of cardiac muscle cell apoptotic process [GO:0010665] Sources: GOC:dph, GOC:mtg_apoptosis, GOC:tb Relationships: is a type of regulation of muscle cell apoptotic process [GO:0010660]; regulates striated muscle cell apoptotic process [GO:0010658] Also known as: regulation of striated muscle cell apoptosis Definition: Any process that modulates the rate or extent of striated muscle cell apoptotic process, a form of programmed cell death induced by external or internal signals that trigger the activity of proteolytic caspases whose actions dismantle a striated muscle cell and result in its death.